{
  "gene_name": "Acetylcholinesterase",
  "gene": "UniProtKB:P22303",
  "term_id": "GO:0003990",
  "gene_symbol": "ACHE",
  "term_label": "acetylcholinesterase activity"
}